{
  "gene_symbol": "MYO1C",
  "term_id": "GO:0006897",
  "gene": "UniProtKB:O00159",
  "gene_name": "Unconventional myosin-Ic",
  "term_label": "endocytosis"
}